{
  "gene": "UniProtKB:P82251",
  "term_label": "neutral L-amino acid transmembrane transporter activity",
  "gene_name": "b(0,+)-type amino acid transporter 1",
  "gene_symbol": "SLC7A9",
  "term_id": "GO:0015175"
}